{
  "gene": "UniProtKB:A0A8Q3SIZ7",
  "term_label": "Unknown cellular component",
  "term_id": "UNKNOWN:0003",
  "gene_symbol": "A0A8Q3SIZ7",
  "gene_name": "Uncharacterized protein"
}